CCR1 chemokine receptor binding [GO:0031726] (molecular function) Definition: Binding to a CCR1 chemokine receptor. Relationships: is a type of CCR chemokine receptor binding [GO:0048020] Sources: GOC:mah, GOC:nln Also known as: macrophage inflammatory protein-1 alpha receptor binding, CCR1 chemokine receptor ligand